(+)-epi-alpha-bisabolol catabolic process [GO:1901942] (biological process) Also known as: (+)-epi-alpha-bisabolol breakdown, (+)-epi-alpha-bisabolol catabolism, (+)-epi-alpha-bisabolol degradation Relationships: is a type of sesquiterpenoid catabolic process [GO:0016107] References: PMID:22867794 Sources: GOC:TermGenie Definition: The chemical reactions and pathways resulting in the breakdown of (+)-epi-alpha-bisabolol.